{
  "gene_name": "A-kinase anchor protein 8",
  "term_id": "GO:0016363",
  "term_label": "nuclear matrix",
  "gene": "UniProtKB:O43823",
  "gene_symbol": "AKAP8"
}